sodium ion transmembrane transport [GO:0035725] (biological process) Relationships: is a type of sodium ion transport [GO:0006814]; is a type of monoatomic cation transmembrane transport [GO:0098655] Note: Note that this term is not intended for use in annotating lateral movement within membranes. Also known as: sodium ion membrane transport Subtypes: sodium ion export across plasma membrane [GO:0036376], sodium ion import across plasma membrane [GO:0098719] Sources: GOC:vw Regulation: regulated by regulation of sodium ion transmembrane transport [GO:1902305]; negatively regulated by negative regulation of sodium ion transmembrane transport [GO:1902306]; positively regulated by positive regulation of sodium ion transmembrane transport [GO:1902307] Definition: A process in which a sodium ion is transported from one side of a membrane to the other by means of some agent such as a transporter or pore.